{
  "gene": "UniProtKB:P78504",
  "term_label": "Unknown cellular component",
  "term_id": "UNKNOWN:0003",
  "gene_name": "Protein jagged-1",
  "gene_symbol": "JAG1"
}